other organism part [GO:0044217] (CC) Definition: Any constituent part of a secondary organism with which the first organism is interacting. Relationships: is a type of cellular anatomical structure [GO:0110165] Note: Note that this term is in the subset of terms that should not be used for direct gene product annotation. Instead, select a child term or, if no appropriate child term exists, please request a new term. Direct annotations to this term may be amended during annotation QC. Subtypes: host cellular component [GO:0018995], other organism cell membrane [GO:0044218], symbiont cell surface [GO:0106139] Sources: GOC:jl